{
  "gene_name": "Protein lin-7 homolog A",
  "gene_symbol": "LIN7A",
  "term_label": "basolateral plasma membrane",
  "gene": "UniProtKB:O14910",
  "term_id": "GO:0016323"
}